{
  "term_label": "chloride channel regulator activity",
  "gene_symbol": "BSND",
  "term_id": "GO:0017081",
  "gene": "UniProtKB:Q8WZ55",
  "gene_name": "Barttin"
}